{
  "term_label": "protein secretion",
  "term_id": "GO:0009306",
  "gene_symbol": "CTAGE8",
  "gene_name": "cTAGE family member 8",
  "gene": "UniProtKB:P0CG41"
}